pyruvate fermentation via PFOR [GO:0044813] (biological process) Definition: The anaerobic chemical reactions and pathways resulting in the breakdown of pyruvate via pyruvate:ferredoxin oxidoreductase (PFOR) activity. This pathway is found in strict anaerobes such as Clostridia species. References: PMID:20395274, PMID:20692761 Sources: GOC:mengo_curators Also known as: glycolytic fermentation via PFOR pathway Relationships: is a type of GO:0019660; has part pyruvate synthase activity [GO:0019164]